{
  "gene_symbol": "HSPA1A",
  "term_label": "positive regulation of proteasomal ubiquitin-dependent protein catabolic process",
  "gene": "UniProtKB:P0DMV8",
  "gene_name": "Heat shock 70 kDa protein 1A",
  "term_id": "GO:0032436"
}